{
  "gene_name": "Receptor-type tyrosine-protein phosphatase U",
  "term_label": "Unknown cellular component",
  "gene_symbol": "PTPRU",
  "gene": "UniProtKB:Q92729",
  "term_id": "UNKNOWN:0003"
}